regulation of protein localization by the Cvt pathway [GO:2001159] (biological process) Sources: GOC:obol Also known as: regulation of cytoplasm to vacuole targeting, regulation of cytoplasm-to-vacuole targeting Definition: Any process that modulates the frequency, rate or extent of protein localization by the Cvt pathway. Relationships: is a type of regulation of intracellular protein transport [GO:0033157]; is a type of regulation of vacuolar transport [GO:1903335]; is a type of GO:1903533; regulates cytoplasm to vacuole targeting by the Cvt pathway [GO:0032258]